protein C inhibitor-thrombin complex [GO:0036028] (cellular component) Definition: A heterodimeric protein complex that contains protein C inhibitor (SERPINA5) and thrombin (F2); formation of the complex inhibits the serine protease activity of thrombin. Also known as: PCI-thrombin complex, SERPINA5-thrombin complex, plasma serine protease inhibitor-thrombin complex, protein C inhibitor-F2 complex, protein C inhibitor-coagulation factor II complex, serpin A5-thrombin complex References: PMID:6323392 Sources: GOC:ans Relationships: is a type of serine protease inhibitor complex [GO:0097180]